{
  "gene_name": "Putative uncharacterized protein FLJ36925",
  "gene": "UniProtKB:Q8N9L7",
  "term_label": "Unknown cellular component",
  "gene_symbol": "Q8N9L7",
  "term_id": "UNKNOWN:0003"
}